{
  "gene": "UniProtKB:Q8N668",
  "term_id": "GO:0005768",
  "gene_name": "COMM domain-containing protein 1",
  "gene_symbol": "COMMD1",
  "term_label": "endosome"
}